calcium- and calmodulin-dependent protein kinase complex [GO:0005954] (cellular component) Also known as: CAMK2, calcium/calmodulin-dependent protein kinase complex, CaMKII References: PMID:20668654 Definition: An enzyme complex which in eukaryotes is composed of four different chains: alpha, beta, gamma, and delta. The different isoforms assemble into homo- or heteromultimeric holoenzymes composed of 8 to 12 subunits. Catalyzes the phosphorylation of proteins to O-phosphoproteins. Relationships: is a type of GO:0140535; is a type of catalytic complex [GO:1902494]